{
  "term_label": "Unknown molecular function",
  "term_id": "UNKNOWN:0001",
  "gene_symbol": "ZFYVE28",
  "gene_name": "Lateral signaling target protein 2 homolog",
  "gene": "UniProtKB:Q9HCC9"
}